{
  "term_id": "GO:0050911",
  "gene": "UniProtKB:Q8NGY3",
  "gene_symbol": "OR6K3",
  "gene_name": "Olfactory receptor 6K3",
  "term_label": "detection of chemical stimulus involved in sensory perception of smell"
}